{
  "term_id": "UNKNOWN:0003",
  "term_label": "Unknown cellular component",
  "gene_name": "T cell receptor delta joining 2 (Fragment)",
  "gene": "UniProtKB:A0A075B6V6",
  "gene_symbol": "TRDJ2"
}